{
  "term_id": "GO:0007165",
  "gene": "UniProtKB:Q8NGR2",
  "gene_name": "Olfactory receptor 1L6",
  "term_label": "signal transduction",
  "gene_symbol": "OR1L6"
}